{
  "gene": "UniProtKB:Q5TGY3",
  "term_id": "UNKNOWN:0003",
  "term_label": "Unknown cellular component",
  "gene_symbol": "AHDC1",
  "gene_name": "Transcription factor Gibbin"
}